{
  "term_id": "GO:0005802",
  "term_label": "trans-Golgi network",
  "gene_name": "Phospholipid-transporting ATPase IK",
  "gene": "UniProtKB:O60423",
  "gene_symbol": "ATP8B3"
}